{
  "gene_symbol": "PLD5",
  "gene": "UniProtKB:Q8N7P1",
  "gene_name": "Inactive phospholipase D5",
  "term_id": "UNKNOWN:0001",
  "term_label": "Unknown molecular function"
}